all-trans-octaprenyl-diphosphate synthase activity [GO:0106350] (molecular function) Definition: Catalysis of the reaction: (2E,6E)-farnesyl diphosphate + 5 isopentenyl diphosphate = 5 diphosphate + all-trans-octaprenyl diphosphate. References: PMID:3519603, PMID:8037730 Sources: RHEA:27798 Also known as: terpenyl pyrophosphate synthetase activity, trans-prenyltransferase activity, octaprenyl pyrophosphate synthase activity, trans-heptaprenyltranstransferase activity Relationships: is_a prenyl diphosphate synthase activity [GO:0120531]